{
  "term_id": "GO:0005634",
  "gene_name": "Nitric oxide synthase, inducible",
  "gene_symbol": "NOS2",
  "gene": "UniProtKB:P35228",
  "term_label": "nucleus"
}